{
  "gene_name": "Homeobox protein DLX-4",
  "term_label": "embryonic skeletal system development",
  "term_id": "GO:0048706",
  "gene_symbol": "DLX4",
  "gene": "UniProtKB:Q92988"
}